cardiac neural crest cell differentiation involved in heart development [GO:0061307] (biological process) Definition: The process in which a relatively unspecialized cell acquires specialized features of a cardiac neural crest cell that will migrate to the heart and contribute to its development. Cardiac neural crest cells are specialized cells that migrate toward the heart from the third, fourth and sixth pharyngeal arches. Relationships: is_a GO:0014033; is a type of cardiocyte differentiation [GO:0035051] References: PMID:19705442 Sources: GOC:dph, GOC:mtg_heart